clathrin-sculpted acetylcholine transport vesicle membrane [GO:0060201] (cellular component) Relationships: is a type of transport vesicle membrane [GO:0030658]; is_a clathrin-coated vesicle membrane [GO:0030665]; is part of clathrin-sculpted acetylcholine transport vesicle [GO:0060200] Definition: The lipid bilayer surrounding a clathrin-sculpted acetylcholine transport vesicle. Sources: GOC:dph Also known as: clathrin sculpted acetylcholine constitutive secretory pathway transport vesicle membrane, clathrin sculpted acetylcholine transport vesicle membrane